{
  "gene": "UniProtKB:P09769",
  "gene_name": "Tyrosine-protein kinase Fgr",
  "term_label": "plasma membrane",
  "term_id": "GO:0005886",
  "gene_symbol": "FGR"
}